{
  "gene": "UniProtKB:O75943",
  "gene_symbol": "RAD17",
  "term_label": "mitotic DNA replication checkpoint signaling",
  "term_id": "GO:0033314",
  "gene_name": "Cell cycle checkpoint protein RAD17"
}